{
  "term_id": "GO:0048788",
  "gene": "UniProtKB:Q9UPA5",
  "term_label": "cytoskeleton of presynaptic active zone",
  "gene_symbol": "BSN",
  "gene_name": "Protein bassoon"
}